{
  "gene_symbol": "STK16",
  "term_id": "GO:0005737",
  "gene": "UniProtKB:O75716",
  "term_label": "cytoplasm",
  "gene_name": "Serine_threonine-protein kinase 16"
}